vesicle targeting, cis-Golgi to rough endoplasmic reticulum [GO:0048206] (biological process) Also known as: cis-Golgi to rough ER targeting, cis-Golgi to rough endoplasmic reticulum targeting, vesicle targeting, cis-Golgi to rough ER References: PMID:10219233 Sources: GOC:jid, GOC:mah, ISBN:0716731363 Definition: The process in which vesicles are directed to specific destination membranes during transport from the cis-Golgi to the rough ER. Relationships: is_a retrograde vesicle-mediated transport, Golgi to endoplasmic reticulum [GO:0006890]; is a type of vesicle targeting, to, from or within Golgi [GO:0048199]; is a type of GO:0051650